{
  "term_id": "UNKNOWN:0002",
  "term_label": "Unknown biological process",
  "gene_name": "Leucine-rich repeat neuronal protein 1",
  "gene_symbol": "LRRN1",
  "gene": "UniProtKB:Q6UXK5"
}